{
  "gene_symbol": "EXOSC1",
  "term_id": "GO:0005737",
  "gene": "UniProtKB:Q9Y3B2",
  "term_label": "cytoplasm",
  "gene_name": "Exosome complex component CSL4"
}